{
  "gene_symbol": "DAZ2",
  "term_label": "translation activator activity",
  "gene_name": "Deleted in azoospermia protein 2",
  "gene": "UniProtKB:Q13117",
  "term_id": "GO:0008494"
}